{
  "gene_name": "Zinc finger protein 436",
  "term_id": "GO:0000981",
  "gene": "UniProtKB:Q9C0F3",
  "term_label": "DNA-binding transcription factor activity, RNA polymerase II-specific",
  "gene_symbol": "ZNF436"
}